{
  "gene_symbol": "TRAV29DV5",
  "term_id": "UNKNOWN:0002",
  "gene": "UniProtKB:P04437",
  "gene_name": "T cell receptor alpha variable 29_delta variable 5",
  "term_label": "Unknown biological process"
}